homogentisate phytyltransferase activity [GO:0010176] (molecular function) Also known as: HPT activity Definition: Catalysis of the reaction: homogentisate + phytyl diphosphate + H+ = 2-methyl-6-phytyl-1,4-benzoquinone + CO2 + diphosphate. 2-methyl-6-phytyl-1,4-benzoquinone is also known as 2-methyl-6-phytylplastoquinol. References: PMID:14512521 Sources: MetaCyc:RXN-2541 Relationships: is a type of homogentisate prenyltransferase activity [GO:0010354]